{
  "term_label": "nucleus",
  "gene": "UniProtKB:O94916",
  "term_id": "GO:0005634",
  "gene_name": "Nuclear factor of activated T-cells 5",
  "gene_symbol": "NFAT5"
}